{
  "gene_symbol": "CYP4A11",
  "gene_name": "Cytochrome P450 4A11",
  "term_label": "icosanoid biosynthetic process",
  "gene": "UniProtKB:Q02928",
  "term_id": "GO:0046456"
}